{
  "gene": "UniProtKB:Q9Y3Y4",
  "gene_symbol": "PYGO1",
  "term_label": "spermatid nucleus differentiation",
  "term_id": "GO:0007289",
  "gene_name": "Pygopus homolog 1"
}